abscisic acid binding [GO:0010427] (molecular function) Also known as: ABA binding, abscisate binding Definition: Binding to abscisic acid, a plant hormone that regulates aspects of plant growth. Relationships: is a type of isoprenoid binding [GO:0019840]; is a type of monocarboxylic acid binding [GO:0033293]; is a type of hormone binding [GO:0042562]; is a type of alcohol binding [GO:0043178] References: PMID:17347412